sinus venosus development [GO:0003235] (biological process) Definition: The progression of the sinus venosus over time, from its formation to the mature structure. The sinus venosus is a heart chamber attached to the atrium on the venous side of the embryonic heart. Relationships: is a type of cardiac chamber development [GO:0003205] Sources: GOC:mtg_heart